{
  "gene_name": "RCC1 domain-containing protein 1",
  "term_label": "Unknown molecular function",
  "gene_symbol": "RCCD1",
  "gene": "UniProtKB:A6NED2",
  "term_id": "UNKNOWN:0001"
}